{
  "term_label": "RNA polymerase II cis-regulatory region sequence-specific DNA binding",
  "gene_symbol": "ZBTB2",
  "gene": "UniProtKB:Q8N680",
  "gene_name": "Zinc finger and BTB domain-containing protein 2",
  "term_id": "GO:0000978"
}